{
  "gene_name": "BUB3-interacting and GLEBS motif-containing protein ZNF207",
  "gene": "UniProtKB:O43670",
  "term_label": "nucleus",
  "gene_symbol": "ZNF207",
  "term_id": "GO:0005634"
}